{
  "gene_name": "Adenylate kinase 9",
  "gene": "UniProtKB:Q5TCS8",
  "term_id": "GO:0033862",
  "gene_symbol": "AK9",
  "term_label": "UMP kinase activity"
}